{
  "gene_name": "Olfactory receptor 51D1",
  "gene": "UniProtKB:Q8NGF3",
  "gene_symbol": "OR51D1",
  "term_id": "GO:0005886",
  "term_label": "plasma membrane"
}